{
  "term_label": "cytokine activity",
  "term_id": "GO:0005125",
  "gene_name": "Growth_differentiation factor 15",
  "gene_symbol": "GDF15",
  "gene": "UniProtKB:Q99988"
}